{
  "gene_name": "Mitochondrial transcription rescue factor 1",
  "gene": "UniProtKB:Q9P0P8",
  "term_label": "RNA binding",
  "term_id": "GO:0003723",
  "gene_symbol": "MTRES1"
}